CAK-ERCC2 complex [GO:0070516] (cellular component) Also known as: cyclin-dependent protein kinase activating kinase holoenzyme-ERCC2 complex References: PMID:8692841, PMID:8692842 Definition: A protein complex formed by the association of the cyclin-dependent protein kinase activating kinase (CAK) holoenzyme complex with ERCC2. Relationships: is a type of nuclear protein-containing complex [GO:0140513]